{
  "term_id": "GO:0005634",
  "gene_symbol": "FABP7",
  "gene_name": "Fatty acid-binding protein, brain",
  "term_label": "nucleus",
  "gene": "UniProtKB:O15540"
}